{
  "gene": "UniProtKB:Q9P2H3",
  "term_id": "GO:0005813",
  "term_label": "centrosome",
  "gene_symbol": "IFT80",
  "gene_name": "Intraflagellar transport protein 80 homolog"
}